{
  "gene_symbol": "POU3F3",
  "term_id": "GO:0000978",
  "gene": "UniProtKB:P20264",
  "term_label": "RNA polymerase II cis-regulatory region sequence-specific DNA binding",
  "gene_name": "POU domain, class 3, transcription factor 3"
}